regulation of metanephric mesenchymal cell migration by platelet-derived growth factor receptor-beta signaling pathway [GO:1900238] (biological process) Also known as: regulation of metanephric mesenchymal cell migration by platelet-derived growth factor receptor-beta signalling pathway, regulation of metanephric mesenchyme chemotaxis by platelet-derived growth factor receptor-beta signaling pathway Definition: Any process that modulates the frequency, rate or extent of regulation of metanephric mesenchymal cell migration, by platelet-derived growth factor receptor-beta signaling pathway. Subtypes: positive regulation of metanephric mesenchymal cell migration by platelet-derived growth factor receptor-beta signaling pathway [GO:0035793] References: PMID:19019919 Sources: GOC:TermGenie, GOC:mtg_kidney_jan10, GOC:yaf Relationships: is a type of platelet-derived growth factor receptor-beta signaling pathway [GO:0035791]; is a type of regulation of metanephric mesenchymal cell migration [GO:2000589]